{
  "gene_name": "Sorting nexin-30",
  "gene": "UniProtKB:Q5VWJ9",
  "term_label": "Unknown molecular function",
  "gene_symbol": "SNX30",
  "term_id": "UNKNOWN:0001"
}